{
  "term_id": "GO:0101020",
  "gene_symbol": "CYP3A4",
  "gene_name": "Cytochrome P450 3A4",
  "gene": "UniProtKB:P08684",
  "term_label": "estrogen 16-alpha-hydroxylase activity"
}